{
  "gene": "UniProtKB:O76095",
  "gene_name": "Protein JTB",
  "gene_symbol": "JTB",
  "term_label": "cytoplasm",
  "term_id": "GO:0005737"
}